{
  "term_id": "UNKNOWN:0003",
  "term_label": "Unknown cellular component",
  "gene_symbol": "MIR7-3HG",
  "gene": "UniProtKB:Q8N6C7",
  "gene_name": "Putative uncharacterized protein encoded by MIR7-3HG"
}